{
  "term_label": "signal transduction",
  "gene_name": "Proto-oncogene serine_threonine-protein kinase mos",
  "gene_symbol": "MOS",
  "term_id": "GO:0007165",
  "gene": "UniProtKB:P00540"
}